{
  "gene": "UniProtKB:Q9UKI9",
  "term_label": "DNA-binding transcription factor activity, RNA polymerase II-specific",
  "gene_symbol": "POU2F3",
  "term_id": "GO:0000981",
  "gene_name": "POU domain, class 2, transcription factor 3"
}